{
  "term_label": "G protein-coupled receptor signaling pathway",
  "term_id": "GO:0007186",
  "gene": "UniProtKB:P81277",
  "gene_name": "Prolactin-releasing peptide",
  "gene_symbol": "PRLH"
}